{
  "term_id": "GO:0050919",
  "term_label": "negative chemotaxis",
  "gene_symbol": "SEMA4C",
  "gene_name": "Semaphorin-4C",
  "gene": "UniProtKB:Q9C0C4"
}